{
  "term_label": "Unknown cellular component",
  "gene_name": "Oxidative stress-induced growth inhibitor 1",
  "gene": "UniProtKB:Q9UJX0",
  "gene_symbol": "OSGIN1",
  "term_id": "UNKNOWN:0003"
}